{
  "term_id": "GO:0006783",
  "gene_symbol": "TMEM14B",
  "gene": "UniProtKB:Q9NUH8",
  "term_label": "heme biosynthetic process",
  "gene_name": "Transmembrane protein 14B"
}